plasma membrane lactate transport [GO:0035879] (biological process) Definition: The directed movement of lactate across a plasma membrane. Sources: GOC:mcc Also known as: lactate plasma membrane transport Relationships: is a type of GO:0035873 Subtypes: lactic acid secretion [GO:0046722]